{
  "gene": "UniProtKB:A0A0J9YXY3",
  "term_label": "Unknown molecular function",
  "gene_symbol": "TRBV6-2",
  "gene_name": "T cell receptor beta variable 6-2",
  "term_id": "UNKNOWN:0001"
}